{
  "gene_symbol": "EIF4E2",
  "gene_name": "Eukaryotic translation initiation factor 4E type 2",
  "term_id": "GO:0000340",
  "term_label": "RNA 7-methylguanosine cap binding",
  "gene": "UniProtKB:O60573"
}